{
  "gene_name": "Oxysterol-binding protein-related protein 6",
  "gene": "UniProtKB:Q9BZF3",
  "gene_symbol": "OSBPL6",
  "term_label": "nuclear membrane",
  "term_id": "GO:0031965"
}